{
  "term_label": "synaptic vesicle endocytosis",
  "gene_name": "Alpha-synuclein",
  "gene": "UniProtKB:P37840",
  "gene_symbol": "SNCA",
  "term_id": "GO:0048488"
}